positive regulation of initiation of premeiotic DNA replication [GO:1904514] (biological process) Relationships: is a type of positive regulation of nuclear cell cycle DNA replication [GO:0010571]; is a type of positive regulation of DNA-templated DNA replication initiation [GO:0032298]; is a type of GO:1904512; is a type of positive regulation of reproductive process [GO:2000243]; positively regulates meiotic DNA replication initiation [GO:1902974] Also known as: positive regulation of premeiotic DNA replication initiation, up regulation of initiation of premeiotic DNA replication, up regulation of premeiotic DNA replication initiation, up-regulation of initiation of premeiotic DNA replication, up-regulation of premeiotic DNA replication initiation, upregulation of initiation of premeiotic DNA replication, upregulation of premeiotic DNA replication initiation, activation of initiation of premeiotic DNA replication, activation of premeiotic DNA replication initiation, activation of initiation of meiotic DNA synthesis, activation of initiation of premeiotic DNA synthesis, activation of meiotic DNA replication initiation, positive regulation of initiation of meiotic DNA synthesis, positive regulation of initiation of premeiotic DNA synthesis, positive regulation of meiotic DNA replication initiation, up regulation of initiation of meiotic DNA synthesis, up regulation of initiation of premeiotic DNA synthesis, up regulation of meiotic DNA replication initiation, up-regulation of initiation of meiotic DNA synthesis, up-regulation of initiation of premeiotic DNA synthesis, up-regulation of meiotic DNA replication initiation, upregulation of initiation of meiotic DNA synthesis, upregulation of initiation of premeiotic DNA synthesis, upregulation of meiotic DNA replication initiation Definition: Any process that activates or increases the frequency, rate or extent of initiation of premeiotic DNA replication. References: PMID:25891897 Sources: GOC:TermGenie, GO_REF:0000058